fatty acid ligase activity [GO:0015645] (molecular function) Relationships: is a type of acid-thiol ligase activity [GO:0016878]; is_a ATP-dependent activity [GO:0140657] Subtypes: long-chain fatty acid [acyl-carrier-protein] ligase activity [GO:0008922], long-chain fatty acid--protein ligase activity [GO:0047474], fatty acid-CoA ligase activity [GO:0120515] Definition: Catalysis of the ligation of a fatty acid to an acceptor, coupled to the hydrolysis of ATP. Also known as: fatty-acid ligase activity, fatty acid CoA ligase activity, fatty acyl-coenzyme A synthetase activity Sources: GOC:cjk, GOC:mah